{
  "gene_symbol": "ZNF705B",
  "gene": "UniProtKB:P0CI00",
  "gene_name": "Putative zinc finger protein 705B",
  "term_id": "GO:0005634",
  "term_label": "nucleus"
}